{
  "gene": "UniProtKB:Q13002",
  "term_id": "GO:0098839",
  "gene_name": "Glutamate receptor ionotropic, kainate 2",
  "gene_symbol": "GRIK2",
  "term_label": "postsynaptic density membrane"
}